{
  "term_id": "UNKNOWN:0003",
  "gene_name": "Keratin-associated protein 5-9",
  "gene": "UniProtKB:P26371",
  "gene_symbol": "KRTAP5-9",
  "term_label": "Unknown cellular component"
}